cellular response to methylglyoxal [GO:0097238] (biological process) Definition: Any process that results in a change in state or activity of a cell (in terms of movement, secretion, enzyme production, gene expression, etc.) as a result of a methylglyoxal stimulus. Methylglyoxal is a 2-oxoaldehyde derived from propanal. Relationships: is a type of response to methylglyoxal [GO:0051595]; is a type of GO:0110096; is a type of cellular response to ketone [GO:1901655] Sources: GOC:pr